{
  "term_label": "early endosome",
  "term_id": "GO:0005769",
  "gene_name": "Protein phosphatase 1 regulatory subunit 21",
  "gene": "UniProtKB:Q6ZMI0",
  "gene_symbol": "PPP1R21"
}